{
  "term_id": "GO:0006891",
  "gene": "UniProtKB:Q53S08",
  "gene_name": "Ras-related protein Rab-6D",
  "gene_symbol": "RAB6D",
  "term_label": "intra-Golgi vesicle-mediated transport"
}